{
  "term_id": "GO:0007178",
  "term_label": "cell surface receptor protein serine/threonine kinase signaling pathway",
  "gene_name": "Growth_differentiation factor 9",
  "gene": "UniProtKB:O60383",
  "gene_symbol": "GDF9"
}